regulation of ent-pimara-8(14),15-diene biosynthetic process [GO:1901542] (biological process) Subtypes: GO:1901543, GO:1901544 Also known as: regulation of ent-pimara-8(14),15-diene anabolism, regulation of ent-pimara-8(14),15-diene biosynthesis, regulation of ent-pimara-8(14),15-diene formation, regulation of ent-pimara-8(14),15-diene synthesis Sources: GOC:TermGenie, GOC:di Definition: Any process that modulates the frequency, rate or extent of ent-pimara-8(14),15-diene biosynthetic process. Relationships: is_a regulation of isoprenoid metabolic process [GO:0019747]; is a type of regulation of lipid biosynthetic process [GO:0046890]; regulates ent-pimara-8(14),15-diene biosynthetic process [GO:1901541]